{
  "gene": "UniProtKB:P54652",
  "term_label": "ATP hydrolysis activity",
  "gene_symbol": "HSPA2",
  "gene_name": "Heat shock-related 70 kDa protein 2",
  "term_id": "GO:0016887"
}